{
  "gene_symbol": "SCG2",
  "gene": "UniProtKB:P13521",
  "gene_name": "Secretogranin-2",
  "term_id": "GO:0005125",
  "term_label": "cytokine activity"
}